{
  "gene": "UniProtKB:P30085",
  "gene_symbol": "CMPK1",
  "gene_name": "UMP-CMP kinase",
  "term_id": "GO:0033862",
  "term_label": "UMP kinase activity"
}